cytoplasmic dynein complex [GO:0005868] (cellular component) Definition: Any dynein complex with a homodimeric dynein heavy chain core that catalyzes movement along a microtubule. Cytoplasmic dynein complexes participate in many cytoplasmic transport activities in eukaryotes, such as mRNA localization, intermediate filament transport, nuclear envelope breakdown, apoptosis, transport of centrosomal proteins, mitotic spindle assembly, virus transport, kinetochore functions, and movement of signaling and spindle checkpoint proteins. Some complexes participate in intraflagellar transport. Subunits associated with the dynein heavy chain mediate association between dynein heavy chain and cargoes, and may include light chains and light intermediate chains. References: PMID:12600311 Sources: GOC:cilia, GOC:hla, GOC:krc, GOC:mah Also known as: cytoplasmic dynein heavy chain, cytoplasmic dynein intermediate chain, cytoplasmic dynein intermediate light chain, cytoplasmic dynein light chain Note: Note that this term is labelled based on phylogenetic classification and community usage, rather than strict cellular localization. Cytoplasmic dynein complexes may contain ciliary dyneins; therefore the term is not linked to 'cytoplasm'. Cytoplasmic dynein complexes do not contain axonemal dyneins; see GO:0005858 axonemal dynein complex. Relationships: is a type of GO:0030286